inhibitory postsynaptic potential [GO:0060080] (biological process) Definition: A process that causes a temporary decrease in postsynaptic membrane potential due to the flow of negatively charged ions into the postsynaptic cell. The flow of ions that causes an IPSP is an inhibitory postsynaptic current (IPSC) and makes it more difficult for the neuron to fire an action potential. Regulation: positively regulated by positive regulation of inhibitory postsynaptic potential [GO:0097151]; regulated by modulation of inhibitory postsynaptic potential [GO:0098828] Relationships: is a type of GO:0060078; BFO_0000050 chemical synaptic transmission, postsynaptic [GO:0099565] Also known as: regulation of inhibitory post-synaptic membrane potential, IPSP Sources: GOC:dph, GOC:ef